{
  "gene_name": "Protein FAM24A",
  "term_id": "UNKNOWN:0003",
  "term_label": "Unknown cellular component",
  "gene_symbol": "FAM24A",
  "gene": "UniProtKB:A6NFZ4"
}